{
  "gene_name": "NACHT, LRR and PYD domains-containing protein 9",
  "gene": "UniProtKB:Q7RTR0",
  "term_id": "GO:0061702",
  "term_label": "canonical inflammasome complex",
  "gene_symbol": "NLRP9"
}